{
  "gene_symbol": "SLC1A2",
  "term_id": "GO:0005886",
  "gene_name": "Excitatory amino acid transporter 2",
  "term_label": "plasma membrane",
  "gene": "UniProtKB:P43004"
}